{
  "gene": "UniProtKB:Q13867",
  "gene_symbol": "BLMH",
  "term_id": "GO:0004177",
  "term_label": "aminopeptidase activity",
  "gene_name": "Bleomycin hydrolase"
}